involuntary skeletal muscle contraction [GO:0003011] (biological process) Definition: A process in which force is generated within involuntary skeletal muscle tissue, resulting in a change in muscle geometry. Force generation involves a chemo-mechanical energy conversion step that is carried out by the actin/myosin complex activity, which generates force through ATP hydrolysis. Involuntary skeletal muscle is skeletal muscle that is not under conscious control. Relationships: is a type of skeletal muscle contraction [GO:0003009] Subtypes: diaphragm contraction [GO:0002086] Sources: GOC:mtg_cardio, GOC:mtg_muscle